{
  "term_id": "GO:0061575",
  "gene": "UniProtKB:Q8ND76",
  "gene_symbol": "CCNY",
  "term_label": "cyclin-dependent protein serine/threonine kinase activator activity",
  "gene_name": "Cyclin-Y"
}